clathrin-coated endocytic vesicle membrane [GO:0030669] (cellular component) Definition: The lipid bilayer surrounding a clathrin-coated endocytic vesicle. Sources: GOC:mah Relationships: is a type of clathrin-coated vesicle membrane [GO:0030665]; is a type of endocytic vesicle membrane [GO:0030666]; is part of clathrin-coated endocytic vesicle [GO:0045334] Subtypes: GO:0030671